{
  "gene": "UniProtKB:Q6K0P9",
  "gene_symbol": "PYHIN1",
  "term_id": "GO:0005829",
  "gene_name": "Pyrin and HIN domain-containing protein 1",
  "term_label": "cytosol"
}